{
  "gene": "UniProtKB:Q9NX76",
  "gene_symbol": "CMTM6",
  "term_id": "GO:0016020",
  "term_label": "membrane",
  "gene_name": "CKLF-like MARVEL transmembrane domain-containing protein 6"
}